plant organ morphogenesis [GO:1905392] (biological process) Relationships: is a type of GO:0009653; is part of plant organ development [GO:0099402] Definition: The developmental process by which a plant organ is generated and organized. Subtypes: leaf morphogenesis [GO:0009965], GO:0010015, bract morphogenesis [GO:0010433], plant ovule morphogenesis [GO:0048482], post-embryonic plant organ morphogenesis [GO:0090697] Sources: GOC:TermGenie, GOC:tb, GO_REF:0000083 Regulation: regulated by GO:1905421; negatively regulated by negative regulation of plant organ morphogenesis [GO:1905422]; positively regulated by GO:1905423